ureidoglycolate hydrolase activity [GO:0004848] (molecular function) Note: Take care to annotate to the reaction, not simply the enzyme name. The name "ureidoglycolate hydrolase" has variously been used to refer to two distinctly different enzymes. Both enzymes act on ureidoglycolate and produce glyoxylate, but the mechanism and reaction products are different. The "ureidoglycolate hydrolase" listed in the Enzyme commission (EC) is a ureidoglycolate amidohydrolase, releasing ammonia, (EC:3.5.1.116, GO:0004848). The "ureidoglycolate hydrolase" characterized in PMID:3915539 (published prior to the EC designation of EC:3.5.1.116) is a ureidoglycolate lyase, releasing urea (EC:4.3.2.3, GO:0050385). The inappropriate labelling of ureidoglycolate lyase as EC:3.5.1.116 has caused much confusion in the literature (see PMID:24107613). Take care to correctly annotate based on the reaction products, rather than name. Relationships: is a type of hydrolase activity, acting on carbon-nitrogen (but not peptide) bonds, in linear amides [GO:0016811] Sources: RHEA:19809 Also known as: ureidoglycolate amidohydrolase activity Definition: Catalysis of the reaction: (S)-ureidoglycolate + H2O + 2 H+ = CO2 + glyoxylate + 2 NH4.